{
  "term_id": "UNKNOWN:0002",
  "gene_name": "DnaJ homolog subfamily C member 8",
  "gene": "UniProtKB:O75937",
  "term_label": "Unknown biological process",
  "gene_symbol": "DNAJC8"
}